{
  "gene_symbol": "CHRNB4",
  "term_label": "acetylcholine receptor signaling pathway",
  "gene": "UniProtKB:P30926",
  "term_id": "GO:0095500",
  "gene_name": "Neuronal acetylcholine receptor subunit beta-4"
}